regulation of neuron maturation [GO:0014041] (biological process) Definition: Any process that modulates the frequency, rate or extent of neuron maturation, the process leading to the attainment of the full functional capacity of a neuron. This process is independent of morphogenetic change. Sources: GOC:ef Relationships: is a type of GO:0045664; is a type of GO:1903429; regulates GO:0042551 Subtypes: positive regulation of neuron maturation [GO:0014042], negative regulation of neuron maturation [GO:0014043], regulation of neuron remodeling [GO:1904799]